{
  "gene_name": "Eukaryotic translation initiation factor 4E type 1B",
  "term_label": "translational initiation",
  "gene_symbol": "EIF4E1B",
  "gene": "UniProtKB:A6NMX2",
  "term_id": "GO:0006413"
}